{
  "gene_symbol": "CRYGN",
  "term_label": "structural constituent of eye lens",
  "gene_name": "Gamma-crystallin N",
  "gene": "UniProtKB:Q8WXF5",
  "term_id": "GO:0005212"
}